{
  "term_id": "GO:0005634",
  "term_label": "nucleus",
  "gene_symbol": "FAM53C",
  "gene_name": "Protein FAM53C",
  "gene": "UniProtKB:Q9NYF3"
}